1,3-beta-glucanosyltransferase activity [GO:0042124] (molecular function) Definition: Catalysis of the splitting and linkage of (1->3)-beta-D-glucan molecules, resulting in (1->3)-beta-D-glucan chain elongation. References: PMID:10809732 Sources: GOC:jl Relationships: is a type of glucanosyltransferase activity [GO:0042123]